{
  "gene_name": "Olfactory receptor 10K2",
  "gene_symbol": "OR10K2",
  "term_id": "GO:0050911",
  "term_label": "detection of chemical stimulus involved in sensory perception of smell",
  "gene": "UniProtKB:Q6IF99"
}